{
  "gene_symbol": "MKNK2",
  "term_id": "GO:0035556",
  "gene_name": "MAP kinase-interacting serine_threonine-protein kinase 2",
  "gene": "UniProtKB:Q9HBH9",
  "term_label": "intracellular signal transduction"
}